{
  "term_id": "GO:0008201",
  "gene_name": "Epididymal sperm-binding protein 1",
  "term_label": "heparin binding",
  "gene_symbol": "ELSPBP1",
  "gene": "UniProtKB:Q96BH3"
}